{
  "gene": "UniProtKB:O43291",
  "gene_name": "Kunitz-type protease inhibitor 2",
  "term_id": "GO:0007163",
  "term_label": "establishment or maintenance of cell polarity",
  "gene_symbol": "SPINT2"
}